{
  "gene": "UniProtKB:P18507",
  "gene_symbol": "GABRG2",
  "term_label": "dendrite membrane",
  "gene_name": "Gamma-aminobutyric acid receptor subunit gamma-2",
  "term_id": "GO:0032590"
}